{
  "term_label": "DNA methylation-dependent constitutive heterochromatin formation",
  "term_id": "GO:0006346",
  "gene_name": "Methyl-CpG-binding domain protein 1",
  "gene": "UniProtKB:Q9UIS9",
  "gene_symbol": "MBD1"
}